{
  "gene": "UniProtKB:P68032",
  "gene_name": "Actin, alpha cardiac muscle 1",
  "gene_symbol": "ACTC1",
  "term_label": "actin filament organization",
  "term_id": "GO:0007015"
}